{
  "term_id": "GO:0009435",
  "term_label": "NAD+ biosynthetic process",
  "gene_symbol": "NADSYN1",
  "gene_name": "Glutamine-dependent NAD(+) synthetase",
  "gene": "UniProtKB:Q6IA69"
}